{
  "term_id": "GO:0006338",
  "term_label": "chromatin remodeling",
  "gene_name": "Lysine-specific demethylase 2A",
  "gene_symbol": "KDM2A",
  "gene": "UniProtKB:Q9Y2K7"
}